cochlea morphogenesis [GO:0090103] (biological process) Definition: The process in which the cochlea is generated and organized. Sources: GOC:dph, GOC:tb Relationships: is a type of GO:0048598; is part of GO:0042472; is part of cochlea development [GO:0090102]